{
  "term_id": "GO:0030154",
  "term_label": "cell differentiation",
  "gene": "UniProtKB:Q5JSZ5",
  "gene_symbol": "PRRC2B",
  "gene_name": "Protein PRRC2B"
}